{
  "gene_symbol": "IFT70B",
  "term_label": "axonemal microtubule",
  "gene_name": "Intraflagellar transport protein 70B",
  "gene": "UniProtKB:Q8N4P2",
  "term_id": "GO:0005879"
}